{
  "term_label": "Unknown molecular function",
  "gene_symbol": "PRR5",
  "term_id": "UNKNOWN:0001",
  "gene": "UniProtKB:P85299",
  "gene_name": "Proline-rich protein 5"
}